{
  "gene_symbol": "KCNA1",
  "gene_name": "Potassium voltage-gated channel subfamily A member 1",
  "term_id": "GO:0033270",
  "term_label": "paranode region of axon",
  "gene": "UniProtKB:Q09470"
}